{
  "term_label": "ERAD pathway",
  "term_id": "GO:0036503",
  "gene_name": "Calreticulin-3",
  "gene": "UniProtKB:Q96L12",
  "gene_symbol": "CALR3"
}